{
  "term_id": "GO:0002250",
  "gene_symbol": "BMX",
  "gene_name": "Cytoplasmic tyrosine-protein kinase BMX",
  "term_label": "adaptive immune response",
  "gene": "UniProtKB:P51813"
}